{
  "gene_name": "Endogenous retrovirus group K member 24 Gag polyprotein",
  "term_id": "UNKNOWN:0002",
  "term_label": "Unknown biological process",
  "gene": "UniProtKB:P63145",
  "gene_symbol": "ERVK-24"
}